{
  "gene_symbol": "NUMBL",
  "term_id": "GO:0050769",
  "gene_name": "Numb-like protein",
  "term_label": "positive regulation of neurogenesis",
  "gene": "UniProtKB:Q9Y6R0"
}